{
  "gene": "UniProtKB:Q13753",
  "term_id": "UNKNOWN:0003",
  "gene_symbol": "LAMC2",
  "term_label": "Unknown cellular component",
  "gene_name": "Laminin subunit gamma-2"
}